{
  "term_label": "intracellular protein transport",
  "gene_symbol": "ARL14",
  "term_id": "GO:0006886",
  "gene": "UniProtKB:Q8N4G2",
  "gene_name": "ADP-ribosylation factor-like protein 14"
}